{
  "gene_name": "Proline-rich protein 20A",
  "term_id": "UNKNOWN:0001",
  "gene": "UniProtKB:P86496",
  "gene_symbol": "PRR20A",
  "term_label": "Unknown molecular function"
}